positive regulation of type B pancreatic cell development [GO:2000078] (biological process) Definition: Any process that activates or increases the frequency, rate or extent of pancreatic B cell development. Sources: GOC:obol, GOC:yaf Relationships: is a type of positive regulation of cell development [GO:0010720]; is_a positive regulation of epithelial cell differentiation [GO:0030858]; is a type of positive regulation of multicellular organismal process [GO:0051240]; is a type of regulation of type B pancreatic cell development [GO:2000074]; positively regulates GO:0003323 Also known as: positive regulation of pancreatic B cell development, positive regulation of pancreatic beta cell development